{
  "gene_symbol": "EVL",
  "term_label": "plasma membrane",
  "term_id": "GO:0005886",
  "gene_name": "Ena_VASP-like protein",
  "gene": "UniProtKB:Q9UI08"
}